{
  "gene_symbol": "PPARD",
  "term_id": "GO:0001227",
  "term_label": "DNA-binding transcription repressor activity, RNA polymerase II-specific",
  "gene_name": "Peroxisome proliferator-activated receptor delta",
  "gene": "UniProtKB:Q03181"
}